{
  "gene_symbol": "CSF1R",
  "gene_name": "Macrophage colony-stimulating factor 1 receptor",
  "gene": "UniProtKB:P07333",
  "term_label": "growth factor binding",
  "term_id": "GO:0019838"
}